{
  "gene": "UniProtKB:O00560",
  "term_id": "GO:0005886",
  "gene_name": "Syntenin-1",
  "term_label": "plasma membrane",
  "gene_symbol": "SDCBP"
}